{
  "gene_symbol": "PARP2",
  "gene": "UniProtKB:Q9UGN5",
  "term_label": "NAD+-protein-glutamate ADP-ribosyltransferase activity",
  "term_id": "GO:0140807",
  "gene_name": "Poly [ADP-ribose] polymerase 2"
}